2-furoate-CoA ligase activity [GO:0047541] (molecular function) Definition: Catalysis of the reaction: 2-furoate + ATP + CoA = 2-furoyl-CoA + AMP + diphosphate + H+. Sources: EC:6.2.1.31, RHEA:19269 Relationships: is a type of CoA-ligase activity [GO:0016405]; is a type of acid-thiol ligase activity [GO:0016878] Also known as: 2-furoate:CoA ligase (AMP-forming), 2-furoyl coenzyme A synthetase activity